negative regulation of astral microtubule depolymerization [GO:0032932] (biological process) Relationships: is a type of GO:0007026; is a type of negative regulation of cell cycle process [GO:0010948]; is a type of regulation of spindle organization [GO:0090224]; negatively regulates astral microtubule depolymerization [GO:0060172] Also known as: astral microtubule stabilization Sources: GOC:mah Definition: Any process that stops, prevents, or reduces the frequency, rate or extent of the depolymerization of astral microtubules.